positive regulation of aflatoxin biosynthetic process [GO:1900179] (biological process) Definition: Any process that activates or increases the frequency, rate or extent of aflatoxin biosynthetic process. Relationships: is a type of positive regulation of small molecule metabolic process [GO:0062013]; is a type of regulation of aflatoxin biosynthetic process [GO:1900177]; is a type of positive regulation of secondary metabolite biosynthetic process [GO:1900378]; positively regulates GO:0045122 Sources: GOC:di Also known as: positive regulation of aflatoxin anabolism, positive regulation of aflatoxin biosynthesis, positive regulation of aflatoxin formation, positive regulation of aflatoxin synthesis, up regulation of aflatoxin anabolism, up regulation of aflatoxin biosynthesis, up regulation of aflatoxin biosynthetic process, up regulation of aflatoxin formation, up regulation of aflatoxin synthesis, up-regulation of aflatoxin anabolism, up-regulation of aflatoxin biosynthesis, up-regulation of aflatoxin biosynthetic process, up-regulation of aflatoxin formation, up-regulation of aflatoxin synthesis, upregulation of aflatoxin anabolism, upregulation of aflatoxin biosynthesis, upregulation of aflatoxin biosynthetic process, upregulation of aflatoxin formation, upregulation of aflatoxin synthesis, activation of aflatoxin anabolism, activation of aflatoxin biosynthesis, activation of aflatoxin biosynthetic process, activation of aflatoxin formation, activation of aflatoxin synthesis